urease activator activity [GO:0018237] (molecular function) Relationships: is a type of enzyme activator activity [GO:0008047]; RO_0002213 GO:0009039 Also known as: urease activase activity References: PMID:16244137 Sources: GOC:mah Definition: Increases the activity of urease by promoting the incorporation of nickel into the active site.